{
  "gene": "UniProtKB:Q9NR99",
  "term_label": "Unknown cellular component",
  "term_id": "UNKNOWN:0003",
  "gene_name": "Matrix-remodeling-associated protein 5",
  "gene_symbol": "MXRA5"
}